{
  "gene_name": "Tachykinin-4",
  "term_id": "GO:0031835",
  "gene": "UniProtKB:Q86UU9",
  "term_label": "substance P receptor binding",
  "gene_symbol": "TAC4"
}